{
  "term_label": "neuron projection",
  "gene_name": "Neurensin-1",
  "term_id": "GO:0043005",
  "gene": "UniProtKB:Q8IZ57",
  "gene_symbol": "NRSN1"
}